{
  "gene_name": "Putative uncharacterized protein C1orf140",
  "gene_symbol": "C1orf140",
  "gene": "UniProtKB:Q5VVS0",
  "term_label": "Unknown biological process",
  "term_id": "UNKNOWN:0002"
}